{
  "gene": "UniProtKB:Q13023",
  "gene_symbol": "AKAP6",
  "term_id": "GO:0010880",
  "term_label": "regulation of release of sequestered calcium ion into cytosol by sarcoplasmic reticulum",
  "gene_name": "A-kinase anchor protein 6"
}